{
  "gene_symbol": "PSMB4",
  "term_id": "GO:0005829",
  "gene": "UniProtKB:P28070",
  "gene_name": "Proteasome subunit beta type-4",
  "term_label": "cytosol"
}